{
  "gene_symbol": "MAFB",
  "term_id": "GO:0005634",
  "gene_name": "Transcription factor MafB",
  "gene": "UniProtKB:Q9Y5Q3",
  "term_label": "nucleus"
}